specification of ovule identity [GO:0010622] (biological process) Definition: The regionalization process in which the identity of an ovule is specified. Identity is considered to be the aggregate of characteristics by which a structure is recognized. Sources: GOC:tb Relationships: is a type of regionalization [GO:0003002]; is_a developmental process involved in reproduction [GO:0003006]; is part of plant ovule morphogenesis [GO:0048482]